{
  "gene": "UniProtKB:Q8WXF0",
  "term_id": "GO:0003729",
  "gene_name": "Serine_arginine-rich splicing factor 12",
  "gene_symbol": "SRSF12",
  "term_label": "mRNA binding"
}